{
  "term_label": "Unknown biological process",
  "gene_symbol": "SERHL2",
  "gene": "UniProtKB:Q9H4I8",
  "term_id": "UNKNOWN:0002",
  "gene_name": "Serine hydrolase-like protein 2"
}